{
  "gene_name": "Cytochrome b-c1 complex subunit 6-like, mitochondrial",
  "gene": "UniProtKB:A0A096LP55",
  "term_label": "mitochondrial electron transport, ubiquinol to cytochrome c",
  "term_id": "GO:0006122",
  "gene_symbol": "UQCRHL"
}